natural killer cell differentiation [GO:0001779] (biological process) Regulation: regulated by regulation of natural killer cell differentiation [GO:0032823]; RO_0002212 by GO:0032824; positively regulated by positive regulation of natural killer cell differentiation [GO:0032825] Relationships: is a type of lymphocyte differentiation [GO:0030098]; is a type of natural killer cell activation [GO:0030101] Also known as: NK cell differentiation, natural killer cell development Definition: The process in which a relatively unspecialized cell acquires the specialized features of a natural killer cell. Subtypes: GO:0002325 Sources: GOC:add, ISBN:0781735149 Note: Note that immunologists typically use the word 'development' to refer to cells of B or T cell lineages undergoing the process that GO describes as 'cell differentiation'.